{
  "term_id": "GO:0003723",
  "term_label": "RNA binding",
  "gene_symbol": "SF3B4",
  "gene_name": "Splicing factor 3B subunit 4",
  "gene": "UniProtKB:Q15427"
}